{
  "gene_name": "Uroplakin-2",
  "term_label": "Unknown molecular function",
  "gene_symbol": "UPK2",
  "term_id": "UNKNOWN:0001",
  "gene": "UniProtKB:O00526"
}